ABC-type heme transporter activity [GO:0015439] (molecular function) Definition: Catalysis of the reaction: ATP + H2O + heme(in) = ADP + phosphate + heme(out). Relationships: is a type of GO:0015232; is a type of ABC-type transporter activity [GO:0140359]; is part of heme transmembrane transport [GO:0035351] Also known as: ATP-dependent heme transmembrane transporter activity, haem-transporting ATPase activity, heme-transporting ATPase activity, heme ABC transporter, ATPase-coupled heme transmembrane transporter activity, ATPase-coupled heme transporter activity, protoheme IX ABC transporter activity Sources: RHEA:19261